acetate-CoA ligase (ADP-forming) activity [GO:0043758] (molecular function) Definition: Catalysis of the reaction: ATP + acetate + CoA = ADP + phosphate + acetyl-CoA. Relationships: is a type of acid-thiol ligase activity [GO:0016878] Sources: RHEA:15081 Also known as: acetate thiokinase activity, acetate--CoA ligase (ADP-forming) activity, acetyl coenzyme A synthetase (adenosine diphosphate-forming), acetate:CoA ligase (ADP-forming), acetyl-CoA synthetase (ADP-forming) activity, aryl-CoA synthetase (ADP-forming) activity